{
  "term_id": "GO:0036159",
  "gene_symbol": "CCDC39",
  "term_label": "inner dynein arm assembly",
  "gene": "UniProtKB:Q9UFE4",
  "gene_name": "Coiled-coil domain-containing protein 39"
}